{
  "gene_symbol": "VWF",
  "gene_name": "von Willebrand factor",
  "gene": "UniProtKB:P04275",
  "term_id": "GO:0005201",
  "term_label": "extracellular matrix structural constituent"
}